{
  "term_label": "Unknown cellular component",
  "gene_name": "IQ domain-containing protein F6",
  "term_id": "UNKNOWN:0003",
  "gene_symbol": "IQCF6",
  "gene": "UniProtKB:A8MYZ5"
}